positive regulation of antifungal peptide production [GO:0002804] (biological process) Also known as: up regulation of antifungal peptide production, up-regulation of antifungal peptide production, upregulation of antifungal peptide production, activation of antifungal peptide production, stimulation of antifungal peptide production Definition: Any process that activates or increases the frequency, rate, or extent of antifungal peptide production. Sources: GOC:add Subtypes: positive regulation of antifungal peptide secretion [GO:0002802], positive regulation of antifungal peptide biosynthetic process [GO:0006967] Relationships: is_a positive regulation of antimicrobial peptide production [GO:0002225]; is_a regulation of antifungal peptide production [GO:0002788]; positively regulates antifungal peptide production [GO:0002781]